molybdenum incorporation into metallo-sulfur cluster [GO:0018289] (biological process) Relationships: is a type of metal incorporation into metallo-sulfur cluster [GO:0018282] Definition: The incorporation of molybdenum into a metallo-sulfur cluster. Subtypes: molybdenum incorporation into iron-sulfur cluster [GO:0018291] Sources: GOC:ai Also known as: molybdenum incorporation into metallo-sulphur cluster